regulation of endosome organization [GO:1904978] (biological process) Definition: Any process that modulates the frequency, rate or extent of endosome organization. References: PMID:22511594 Sources: GOC:PARL, GOC:TermGenie, GOC:pad, GO_REF:0000058 Also known as: regulation of endosome organisation, regulation of endosome organization and biogenesis Relationships: is a type of GO:0033043; regulates endosome organization [GO:0007032] Subtypes: GO:1904979, positive regulation of endosome organization [GO:1904980], regulation of intralumenal vesicle formation [GO:1905365]